{
  "gene_symbol": "CDK5RAP3",
  "term_label": "ubiquitin-like ligase-substrate adaptor activity",
  "term_id": "GO:1990756",
  "gene": "UniProtKB:Q96JB5",
  "gene_name": "CDK5 regulatory subunit-associated protein 3"
}